{
  "gene_name": "Periodic tryptophan protein 1 homolog",
  "gene": "UniProtKB:Q13610",
  "term_id": "GO:1990889",
  "gene_symbol": "PWP1",
  "term_label": "histone H4K20me3 reader activity"
}